negative regulation of thyroid hormone generation [GO:2000610] (biological process) Relationships: is a type of negative regulation of hormone metabolic process [GO:0032351]; is a type of regulation of thyroid hormone generation [GO:2000609]; negatively regulates GO:0006590 Sources: GOC:obol Definition: Any process that stops, prevents or reduces the frequency, rate or extent of thyroid hormone generation.